{
  "term_id": "GO:0030036",
  "term_label": "actin cytoskeleton organization",
  "gene_symbol": "STARD13",
  "gene_name": "StAR-related lipid transfer protein 13",
  "gene": "UniProtKB:Q9Y3M8"
}